Ku70:Ku80 complex [GO:0043564] (cellular component) References: PMID:12518983 Also known as: Ku70:Ku80 heterodimer Relationships: is a type of nuclear protein-containing complex [GO:0140513] Definition: Heterodimeric protein complex composed of a 70 kDa and a 80 kDa subunit, binds DNA through a channel formed by the heterodimer. Functions in DNA double stranded break repair, chromosome maintenance, transcription regulation, V(D)J recombination, and activation of DNA-PK.